{
  "term_label": "retromer complex",
  "term_id": "GO:0030904",
  "gene": "UniProtKB:Q9UMY4",
  "gene_symbol": "SNX12",
  "gene_name": "Sorting nexin-12"
}